{
  "term_label": "olfactory receptor activity",
  "gene_name": "Olfactory receptor 2H1",
  "gene_symbol": "OR2H1",
  "term_id": "GO:0004984",
  "gene": "UniProtKB:Q9GZK4"
}